granulocyte differentiation [GO:0030851] (biological process) Definition: The process in which a myeloid precursor cell acquires the specialized features of a granulocyte. Granulocytes are a class of leukocytes characterized by the presence of granules in their cytoplasm. These cells are active in allergic immune reactions such as arthritic inflammation and rashes. This class includes basophils, eosinophils and neutrophils. Subtypes: basophil differentiation [GO:0030221], eosinophil differentiation [GO:0030222], GO:0030223 Sources: GOC:ecd, http://life.nthu.edu.tw/~g864204/dict-search1.htm Also known as: granulocyte cell differentiation Relationships: is a type of myeloid leukocyte differentiation [GO:0002573] Regulation: regulated by regulation of granulocyte differentiation [GO:0030852]; negatively regulated by negative regulation of granulocyte differentiation [GO:0030853]; positively regulated by positive regulation of granulocyte differentiation [GO:0030854]